{
  "gene_symbol": "PPHLN1",
  "term_id": "GO:0097355",
  "gene": "UniProtKB:Q8NEY8",
  "gene_name": "Periphilin-1",
  "term_label": "protein localization to heterochromatin"
}